{
  "gene_name": "Gephyrin",
  "gene_symbol": "GPHN",
  "gene": "UniProtKB:Q9NQX3",
  "term_label": "gamma-aminobutyric acid receptor clustering",
  "term_id": "GO:0097112"
}